{
  "term_label": "positive regulation of phagocytosis",
  "gene_name": "Putative high affinity immunoglobulin gamma Fc receptor IB",
  "term_id": "GO:0050766",
  "gene_symbol": "FCGR1BP",
  "gene": "UniProtKB:Q92637"
}